xylitol metabolic process [GO:0051164] (biological process) Note: Note that xylitol is a meso compound, thus there are no L or D-versions. Also known as: xylitol metabolism Subtypes: xylitol catabolic process [GO:0051160] Relationships: is a type of pentitol metabolic process [GO:0019519] Definition: The chemical reactions and pathways involving xylitol, a five-carbon sugar alcohol derived from xylose by reduction of the carbonyl group. It is as sweet as sucrose and is used as a noncariogenic sweetner and as a sugar substitute in diabetic diets. Sources: GOC:ai